regulation of developmental growth [GO:0048638] (biological process) Definition: Any process that modulates the frequency, rate or extent of developmental growth. Sources: GOC:go_curators Relationships: is a type of regulation of growth [GO:0040008]; is a type of regulation of developmental process [GO:0050793]; regulates developmental growth [GO:0048589] Subtypes: regulation of synaptic assembly at neuromuscular junction [GO:0008582], regulation of meristem growth [GO:0010075], regulation of axon extension [GO:0030516], regulation of multicellular organism growth [GO:0040014], regulation of skeletal muscle tissue regeneration [GO:0043416], GO:0045570, regulation of organ growth [GO:0046620], regulation of skeletal muscle tissue growth [GO:0048631], GO:0048639, negative regulation of developmental growth [GO:0048640], regulation of collateral sprouting [GO:0048670], GO:0048686, regulation of unidimensional cell growth [GO:0051510], regulation of mammary gland cord elongation by mammary fat precursor cell-epithelial cell signaling [GO:0060657], regulation of branch elongation involved in ureteric bud branching [GO:0072095], regulation of seed growth [GO:0080113], regulation of convergent extension involved in axis elongation [GO:1901232], regulation of root hair elongation [GO:1902890], GO:1903041, regulation of dendrite extension [GO:1903859], regulation of trophectodermal cell proliferation [GO:1904073], GO:1905041, regulation of cardiac muscle tissue regeneration [GO:1905178], regulation of developmental vegetative growth [GO:1905613], GO:2000387